posterior lateral line nerve development [GO:0048918] (biological process) Definition: The process whose specific outcome is the progression of the posterior lateral line nerve over time, from its formation to the mature structure. The posterior lateral line nerve innervates hair cells of the PLL and projects to an octavolateralis column in the hindbrain that consists of the medial octavolateralis nucleus (MON), the caudal octavolateralis nucleus, and the magnocellular nucleus. Sources: GOC:cls, GOC:dgh, GOC:dph, GOC:jid, GO_REF:0000021 Also known as: PLLN development, caudal lateral line nerve development Relationships: is a type of lateral line nerve development [GO:0048892]; is part of posterior lateral line system development [GO:0048915]